{
  "gene_symbol": "PRDM10",
  "term_id": "GO:0017053",
  "gene": "UniProtKB:Q9NQV6",
  "gene_name": "PR domain zinc finger protein 10",
  "term_label": "transcription repressor complex"
}